{
  "gene": "UniProtKB:H3BPM6",
  "gene_name": "MKRN2 opposite strand protein",
  "gene_symbol": "MKRN2OS",
  "term_id": "UNKNOWN:0001",
  "term_label": "Unknown molecular function"
}